{
  "gene_name": "Serpin B7",
  "term_id": "GO:0005615",
  "gene": "UniProtKB:O75635",
  "term_label": "extracellular space",
  "gene_symbol": "SERPINB7"
}